5'-nucleotidase activity [GO:0008253] (molecular function) Relationships: is_a nucleotidase activity [GO:0008252] Also known as: 5' nucleotidase activity, 5'-AMP nucleotidase, 5'-AMPase, 5'-adenylic phosphatase, AMP phosphatase, AMP phosphohydrolase, AMPase, UMPase, adenosine 5'-phosphatase, adenosine monophosphatase, snake venom 5'-nucleotidase, thimidine monophosphate nucleotidase, uridine 5'-nucleotidase, 5'-mononucleotidase activity, 5'-ribonucleotide phosphohydrolase activity Definition: Catalysis of the reaction: a 5'-ribonucleotide + H2O = a ribonucleoside + phosphate. Sources: EC:3.1.3.5